{
  "gene_symbol": "MMAB",
  "term_label": "Unknown cellular component",
  "gene_name": "Corrinoid adenosyltransferase MMAB",
  "gene": "UniProtKB:Q96EY8",
  "term_id": "UNKNOWN:0003"
}